{
  "gene_symbol": "NDP",
  "term_id": "UNKNOWN:0003",
  "term_label": "Unknown cellular component",
  "gene": "UniProtKB:Q00604",
  "gene_name": "Norrin"
}